{
  "term_id": "GO:0000785",
  "gene_symbol": "GLYR1",
  "gene": "UniProtKB:Q49A26",
  "term_label": "chromatin",
  "gene_name": "Cytokine-like nuclear factor N-PAC"
}